{
  "gene_name": "Paxillin",
  "term_label": "transforming growth factor beta receptor signaling pathway",
  "term_id": "GO:0007179",
  "gene_symbol": "PXN",
  "gene": "UniProtKB:P49023"
}